{
  "gene_symbol": "SQLE",
  "term_label": "sterol biosynthetic process",
  "term_id": "GO:0016126",
  "gene_name": "Squalene monooxygenase",
  "gene": "UniProtKB:Q14534"
}